{
  "term_id": "GO:0007018",
  "gene_name": "Kinesin-like protein KIF22",
  "gene_symbol": "KIF22",
  "term_label": "microtubule-based movement",
  "gene": "UniProtKB:Q14807"
}